{
  "term_id": "GO:0044614",
  "gene_symbol": "NUP98",
  "term_label": "nuclear pore cytoplasmic filaments",
  "gene": "UniProtKB:P52948",
  "gene_name": "Nuclear pore complex protein Nup98-Nup96"
}